{
  "gene_symbol": "RTL3",
  "term_label": "Unknown molecular function",
  "gene": "UniProtKB:Q8N8U3",
  "gene_name": "Retrotransposon Gag-like protein 3",
  "term_id": "UNKNOWN:0001"
}